{
  "term_id": "UNKNOWN:0001",
  "gene": "UniProtKB:Q53R12",
  "gene_name": "Transmembrane 4 L6 family member 20",
  "term_label": "Unknown molecular function",
  "gene_symbol": "TM4SF20"
}